{
  "gene": "UniProtKB:Q8NFP7",
  "gene_name": "Diphosphoinositol polyphosphate phosphohydrolase 3-alpha",
  "gene_symbol": "NUDT10",
  "term_label": "bis(5'-adenosyl)-pentaphosphatase activity",
  "term_id": "GO:0034432"
}